{
  "term_label": "centrosome",
  "gene": "UniProtKB:Q9P2G4",
  "gene_symbol": "MAP10",
  "gene_name": "Microtubule-associated protein 10",
  "term_id": "GO:0005813"
}